dTMP catabolic process [GO:0046074] (BP) Definition: The chemical reactions and pathways resulting in the breakdown of dTMP, deoxyribosylthymine monophosphate. Sources: GOC:go_curators Relationships: is a type of pyrimidine deoxyribonucleoside monophosphate catabolic process [GO:0009178]; is a type of pyrimidine deoxyribonucleotide catabolic process [GO:0009223]; is a type of dTMP metabolic process [GO:0046073] Also known as: dTMP breakdown, dTMP catabolism, dTMP degradation